{
  "term_id": "GO:0005886",
  "gene": "UniProtKB:P04083",
  "gene_symbol": "ANXA1",
  "gene_name": "Annexin A1",
  "term_label": "plasma membrane"
}